{
  "term_id": "UNKNOWN:0002",
  "gene_symbol": "CCDC194",
  "gene_name": "Coiled-coil domain-containing protein 194",
  "term_label": "Unknown biological process",
  "gene": "UniProtKB:A0A1B0GVG4"
}